negative regulation of siRNA processing [GO:1903704] (biological process) Definition: Any process that stops, prevents or reduces the frequency, rate or extent of siRNA processing. References: PMID:19701182 Sources: GOC:BHF, GOC:TermGenie, GOC:nc, GO_REF:0000058 Relationships: is a type of negative regulation of metabolic process [GO:0009892]; is a type of regulation of siRNA processing [GO:0070921]; negatively regulates siRNA processing [GO:0030422] Also known as: down regulation of RNA interference, production of guide RNAs, down regulation of RNA interference, production of siRNA, down regulation of production of guide RNAs involved in RNA interference, down regulation of production of siRNA involved in RNA interference, down-regulation of RNA interference, production of guide RNAs, down-regulation of RNA interference, production of siRNA, down-regulation of production of guide RNAs involved in RNA interference, down-regulation of production of siRNA involved in RNA interference, downregulation of RNA interference, production of guide RNAs, downregulation of RNA interference, production of siRNA, downregulation of production of guide RNAs involved in RNA interference, downregulation of production of siRNA involved in RNA interference, negative regulation of RNA interference, production of guide RNAs, negative regulation of RNA interference, production of siRNA, negative regulation of production of guide RNAs involved in RNA interference, negative regulation of production of siRNA involved in PTGS, negative regulation of production of siRNA involved in RNA interference, inhibition of RNA interference, production of guide RNAs, inhibition of RNA interference, production of siRNA, inhibition of production of guide RNAs involved in RNA interference, inhibition of production of siRNA involved in RNA interference, negative regulation of production of siRNA involved in post-transcriptional gene silencing by RNA, negative regulation of siRNA production